{
  "gene_name": "T cell receptor alpha joining 2 (non-functional) (Fragment)",
  "term_label": "Unknown cellular component",
  "gene_symbol": "TRAJ2",
  "term_id": "UNKNOWN:0003",
  "gene": "UniProtKB:A0A075B6U9"
}